medial ganglionic eminence cell proliferation [GO:0022020] (biological process) Definition: The multiplication or reproduction of medial ganglionic eminence cells, resulting in the expansion of a cell population. Sources: GOC:cls, GOC:dgh, GOC:dph, GOC:jid, GO_REF:0000021 Relationships: is a type of subpallium cell proliferation in forebrain [GO:0022012]